positive regulation of double-strand break repair via homologous recombination [GO:1905168] (biological process) Relationships: is a type of GO:0010569; is a type of GO:0045911; is a type of positive regulation of double-strand break repair [GO:2000781]; positively regulates double-strand break repair via homologous recombination [GO:0000724] Also known as: positive regulation of HDR, positive regulation of HRR, positive regulation of Rad51-dependent recombinational repair, positive regulation of Rhp51-dependent recombinational repair, positive regulation of homologous recombinational repair, positive regulation of homology-directed repair, up regulation of HDR, up regulation of HRR, up regulation of Rad51-dependent recombinational repair, up regulation of Rhp51-dependent recombinational repair, up regulation of double-strand break repair via homologous recombination, up regulation of homologous recombinational repair, up regulation of homology-directed repair, up-regulation of HDR, up-regulation of HRR, up-regulation of Rad51-dependent recombinational repair, up-regulation of Rhp51-dependent recombinational repair, up-regulation of double-strand break repair via homologous recombination, up-regulation of homologous recombinational repair, up-regulation of homology-directed repair, upregulation of HDR, upregulation of HRR, upregulation of Rad51-dependent recombinational repair, upregulation of Rhp51-dependent recombinational repair, upregulation of double-strand break repair via homologous recombination, upregulation of homologous recombinational repair, upregulation of homology-directed repair, activation of HDR, activation of HRR, activation of Rad51-dependent recombinational repair, activation of Rhp51-dependent recombinational repair, activation of double-strand break repair via homologous recombination, activation of homologous recombinational repair, activation of homology-directed repair References: PMID:12023299 Sources: GOC:TermGenie, GO_REF:0000058 Definition: Any process that activates or increases the frequency, rate or extent of double-strand break repair via homologous recombination.